SMAD protein complex [GO:0071141] (cellular component) Also known as: SMAD complex Relationships: is_a protein-containing complex [GO:0032991] Subtypes: GO:0071142, heteromeric SMAD protein complex [GO:0071144] References: PMID:9670020 Sources: GOC:bhm, GOC:mah Definition: A protein complex that consists of only SMAD proteins; may be homomeric or heteromeric. Heteromeric complexes act as transcription factors while homomeric complexes exist but are transcriptionally inactive. Hetero- versus homotrimerization is largely enthalpy driven.